positive regulation of SCF-dependent proteasomal ubiquitin-dependent catabolic process [GO:0062027] (biological process) References: PMID:28007894 Definition: Any process that starts or increases the rate, frequency or extent of SCF-dependent proteasomal ubiquitin-dependent protein catabolic process, the chemical reactions and pathways resulting in the breakdown of a protein or peptide by hydrolysis of its peptide bonds, initiated by the covalent attachment of ubiquitin, with ubiquitin-protein ligation catalyzed by an SCF (Skp1/Cul1/F-box protein) complex, and mediated by the proteasome. Relationships: is a type of positive regulation of proteasomal ubiquitin-dependent protein catabolic process [GO:0032436]; is a type of regulation of SCF-dependent proteasomal ubiquitin-dependent protein catabolic process [GO:0062025]; positively regulates SCF-dependent proteasomal ubiquitin-dependent protein catabolic process [GO:0031146]